{
  "term_id": "GO:0005634",
  "gene": "UniProtKB:Q8IZM8",
  "gene_name": "Zinc finger protein 654",
  "term_label": "nucleus",
  "gene_symbol": "ZNF654"
}